{
  "gene_symbol": "CDKN2B",
  "term_id": "GO:2000045",
  "gene_name": "Cyclin-dependent kinase 4 inhibitor B",
  "term_label": "regulation of G1/S transition of mitotic cell cycle",
  "gene": "UniProtKB:P42772"
}